{
  "gene": "UniProtKB:O14617",
  "gene_symbol": "AP3D1",
  "term_id": "GO:0010008",
  "term_label": "endosome membrane",
  "gene_name": "AP-3 complex subunit delta-1"
}